{
  "gene_symbol": "SUMO1",
  "term_label": "protein tag activity",
  "gene": "UniProtKB:P63165",
  "term_id": "GO:0031386",
  "gene_name": "Small ubiquitin-related modifier 1"
}